UDP-galactose transmembrane transporter activity [GO:0005459] (molecular function) Relationships: is a type of pyrimidine nucleotide-sugar transmembrane transporter activity [GO:0015165]; BFO_0000050 GO:0072334 Definition: Enables the transfer of a UDP-galactose from one side of a membrane to the other. UDP-galactose is a substance composed of galactose in glycosidic linkage with uridine diphosphate. Sources: GOC:ai, GOC:mtg_transport, ISBN:0815340729